{
  "gene": "UniProtKB:Q5TBB1",
  "term_label": "ribonuclease H2 complex",
  "term_id": "GO:0032299",
  "gene_symbol": "RNASEH2B",
  "gene_name": "Ribonuclease H2 subunit B"
}